{
  "term_id": "GO:0000978",
  "gene_name": "Leucine-rich repeat flightless-interacting protein 1",
  "term_label": "RNA polymerase II cis-regulatory region sequence-specific DNA binding",
  "gene": "UniProtKB:Q32MZ4",
  "gene_symbol": "LRRFIP1"
}